{
  "term_label": "intermediate conductance calcium-activated potassium channel activity",
  "gene_name": "Intermediate conductance calcium-activated potassium channel protein 4",
  "gene": "UniProtKB:O15554",
  "term_id": "GO:0022894",
  "gene_symbol": "KCNN4"
}